{
  "gene": "UniProtKB:O15519",
  "term_label": "CD95 death-inducing signaling complex",
  "term_id": "GO:0031265",
  "gene_name": "CASP8 and FADD-like apoptosis regulator",
  "gene_symbol": "CFLAR"
}